{
  "gene": "UniProtKB:P79483",
  "gene_symbol": "HLA-DRB3",
  "gene_name": "HLA class II histocompatibility antigen, DR beta 3 chain",
  "term_label": "lysosomal membrane",
  "term_id": "GO:0005765"
}